{
  "gene": "UniProtKB:Q14542",
  "term_label": "plasma membrane",
  "term_id": "GO:0005886",
  "gene_symbol": "SLC29A2",
  "gene_name": "Equilibrative nucleoside transporter 2"
}